alpha-humulene 10-hydroxylase activity [GO:0102068] (molecular function) Sources: EC:1.14.14.113, GOC:pz Definition: Catalysis of the reaction: (1E,4E,8E)-alpha-humulene + NADPH + O2 + H+ = 10-hydroxy-alpha-humulene + NADP + H2O. Relationships: is a type of oxidoreductase activity, acting on paired donors, with incorporation or reduction of molecular oxygen, NAD(P)H as one donor, and incorporation of one atom of oxygen [GO:0016709]